{
  "term_id": "GO:0070840",
  "gene_symbol": "BICD1",
  "gene": "UniProtKB:Q96G01",
  "term_label": "dynein complex binding",
  "gene_name": "Protein bicaudal D homolog 1"
}